{
  "gene": "UniProtKB:A0A0A0MT78",
  "term_id": "UNKNOWN:0003",
  "term_label": "Unknown cellular component",
  "gene_symbol": "TRBJ2-7",
  "gene_name": "T cell receptor beta joining 2-7"
}